embryonic skeletal limb joint morphogenesis [GO:0036023] (BP) Definition: The process, occurring in the embryo, in which the anatomical structures of a skeletal limb joint are generated and organized. A skeletal limb joint is the connecting structure between the bones of a limb. Relationships: is a type of limb joint morphogenesis [GO:0036022]; is a type of embryonic skeletal joint morphogenesis [GO:0060272]; is part of GO:0030326 Sources: GOC:bf, Wikipedia:Joint